{
  "term_id": "GO:0019957",
  "gene": "UniProtKB:P51684",
  "gene_symbol": "CCR6",
  "term_label": "C-C chemokine binding",
  "gene_name": "C-C chemokine receptor type 6"
}